regulation of AIM2 inflammasome complex assembly [GO:0140971] (biological process) Subtypes: negative regulation of AIM2 inflammasome complex assembly [GO:0140972], positive regulation of AIM2 inflammasome complex assembly [GO:0140973] Relationships: is a type of regulation of protein-containing complex assembly [GO:0043254]; BFO_0000050 regulation of inflammasome-mediated signaling pathway [GO:0141085]; regulates AIM2 inflammasome complex assembly [GO:0140970] References: PMID:33467177 Definition: Any process that modulates the frequency, rate or extent of AIM2 inflammasome complex assembly.